{
  "gene_symbol": "POTEB",
  "gene": "UniProtKB:A0A0A6YYL3",
  "gene_name": "POTE ankyrin domain family member B",
  "term_id": "UNKNOWN:0001",
  "term_label": "Unknown molecular function"
}